{
  "term_label": "cytoplasm",
  "gene_name": "Eukaryotic translation initiation factor 5B",
  "term_id": "GO:0005737",
  "gene_symbol": "EIF5B",
  "gene": "UniProtKB:O60841"
}